regulation of cellular respiration [GO:0043457] (biological process) Definition: Any process that modulates the frequency, rate or extent of cellular respiration, the enzymatic release of energy from organic compounds. Sources: GOC:jl Relationships: is a type of regulation of generation of precursor metabolites and energy [GO:0043467]; RO_0002211 cellular respiration [GO:0045333] Subtypes: GO:1900318, regulation of methane biosynthetic process from trimethylamine [GO:1900330], regulation of methane biosynthetic process from 3-(methylthio)propionic acid [GO:1900333], regulation of methane biosynthetic process from carbon monoxide [GO:1900336], regulation of methane biosynthetic process from formic acid [GO:1900339], regulation of methane biosynthetic process from dimethyl sulfide [GO:1900342], regulation of methane biosynthetic process from methanethiol [GO:1900345], GO:1900348, negative regulation of cellular respiration [GO:1901856], positive regulation of cellular respiration [GO:1901857], regulation of aerobic respiration [GO:1903715]